{
  "gene_symbol": "SPCS3",
  "gene_name": "Signal peptidase complex subunit 3",
  "gene": "UniProtKB:P61009",
  "term_id": "GO:0006465",
  "term_label": "signal peptide processing"
}